{
  "term_label": "Unknown biological process",
  "term_id": "UNKNOWN:0002",
  "gene_name": "Complement C1q and tumor necrosis factor-related protein 9B",
  "gene": "UniProtKB:B2RNN3",
  "gene_symbol": "C1QTNF9B"
}